{
  "term_label": "protein phosphatase regulator activity",
  "gene_symbol": "PPP2R2D",
  "term_id": "GO:0019888",
  "gene": "UniProtKB:Q66LE6",
  "gene_name": "Serine_threonine-protein phosphatase 2A 55 kDa regulatory subunit B delta isoform"
}